fibronectin fibril [GO:0061800] (cellular component) Definition: A supramolecular fiber formed from fibronectin molecules. The fibrils are 5 to 25nm in diameter and can form branched meshworks. Relationships: is a type of supramolecular fiber [GO:0099512]; is part of GO:0031012 References: PMID:20690820 Sources: GOC:dph